{
  "term_id": "GO:0061891",
  "gene_name": "Synaptotagmin-2",
  "gene_symbol": "SYT2",
  "gene": "UniProtKB:Q8N9I0",
  "term_label": "calcium ion sensor activity"
}